regulation of dopamine uptake involved in synaptic transmission [GO:0051584] (biological process) Definition: Any process that modulates the frequency, rate or extent of the directed movement of the catecholamine neurotransmitter dopamine into a cell. Also known as: regulation of dopamine import involved in synaptic transmission Subtypes: negative regulation of dopamine uptake involved in synaptic transmission [GO:0051585], positive regulation of dopamine uptake involved in synaptic transmission [GO:0051586] Relationships: is a type of regulation of catecholamine uptake involved in synaptic transmission [GO:0051940]; regulates dopamine uptake involved in synaptic transmission [GO:0051583] Sources: GOC:ai